{
  "gene_symbol": "ITPR2",
  "gene_name": "Inositol 1,4,5-trisphosphate receptor type 2",
  "term_label": "inositol 1,4,5-trisphosphate-gated calcium channel activity",
  "gene": "UniProtKB:Q14571",
  "term_id": "GO:0005220"
}